{
  "term_id": "UNKNOWN:0003",
  "gene": "UniProtKB:P15289",
  "gene_symbol": "ARSA",
  "gene_name": "Arylsulfatase A",
  "term_label": "Unknown cellular component"
}